{
  "gene_symbol": "HEATR1",
  "gene_name": "HEAT repeat-containing protein 1",
  "term_id": "GO:0034455",
  "gene": "UniProtKB:Q9H583",
  "term_label": "t-UTP complex"
}